{
  "term_id": "GO:0005021",
  "term_label": "vascular endothelial growth factor receptor activity",
  "gene_symbol": "NRP1",
  "gene_name": "Neuropilin-1",
  "gene": "UniProtKB:O14786"
}